{
  "term_label": "interleukin-7 receptor activity",
  "term_id": "GO:0004917",
  "gene_symbol": "IL7R",
  "gene_name": "Interleukin-7 receptor subunit alpha",
  "gene": "UniProtKB:P16871"
}